{
  "gene_symbol": "PRPF40A",
  "term_id": "GO:0005685",
  "gene_name": "Pre-mRNA-processing factor 40 homolog A",
  "gene": "UniProtKB:O75400",
  "term_label": "U1 snRNP"
}